{
  "term_label": "skeletal muscle myosin thick filament assembly",
  "term_id": "GO:0030241",
  "gene": "UniProtKB:O15273",
  "gene_name": "Telethonin",
  "gene_symbol": "TCAP"
}